{
  "gene": "UniProtKB:Q9UBW5",
  "term_label": "phospholipid binding",
  "gene_name": "Bridging integrator 2",
  "gene_symbol": "BIN2",
  "term_id": "GO:0005543"
}